positive regulation of chemokine (C-X-C motif) ligand 1 production [GO:2000340] (biological process) Also known as: positive regulation of CXCL1 production, positive regulation of KC production, positive regulation of SCYB1 production, positive regulation of keratinocyte derived chemokine production Sources: GOC:BHF, GOC:mah Relationships: is a type of positive regulation of chemokine production [GO:0032722]; is_a regulation of chemokine (C-X-C motif) ligand 1 production [GO:2000338]; positively regulates GO:0072566 Definition: Any process that activates or increases the frequency, rate or extent of chemokine (C-X-C motif) ligand 1 production.